{
  "gene": "UniProtKB:Q07820",
  "gene_name": "Induced myeloid leukemia cell differentiation protein Mcl-1",
  "term_id": "GO:0015267",
  "gene_symbol": "MCL1",
  "term_label": "channel activity"
}